RNA polymerase III type 2 promoter sequence-specific DNA binding [GO:0001003] (molecular function) References: PMID:12381659 Sources: GOC:txnOH Definition: Binding to a sequence of DNA that is a part of a type 2 promoter that controls transcription by RNA polymerase III. Type 2 promoters consist of an A box and a B box downstream of the transcription start site within the sequence within the sequence of the mature RNA. Type 2 promoters are found in many tRNA genes as well as in other small RNAs. Relationships: is a type of GO:0000992 Also known as: RNA polymerase III type 2 promoter DNA binding